{
  "term_label": "negative regulation of transcription by RNA polymerase II",
  "gene_name": "Hairy and enhancer of split-related protein HELT",
  "term_id": "GO:0000122",
  "gene_symbol": "HELT",
  "gene": "UniProtKB:A6NFD8"
}